axial cellular bud site selection [GO:0007120] (biological process) Definition: The process of defining the next site of bud emergence adjacent to the last site of bud emergence on a budding cell. Relationships: is a type of GO:0000282; is a type of cell budding [GO:0007114] Sources: GOC:clt Also known as: axial budding, axial bud site selection